{
  "term_id": "GO:0000978",
  "gene_symbol": "RARB",
  "gene": "UniProtKB:P10826",
  "gene_name": "Retinoic acid receptor beta",
  "term_label": "RNA polymerase II cis-regulatory region sequence-specific DNA binding"
}